{
  "gene": "UniProtKB:Q9Y653",
  "term_label": "G protein-coupled receptor signaling pathway",
  "term_id": "GO:0007186",
  "gene_name": "Adhesion G-protein coupled receptor G1",
  "gene_symbol": "ADGRG1"
}